{
  "gene_name": "Zinc finger MYND domain-containing protein 11",
  "gene": "UniProtKB:Q15326",
  "term_label": "nucleus",
  "gene_symbol": "ZMYND11",
  "term_id": "GO:0005634"
}